{
  "term_id": "GO:0005615",
  "gene_symbol": "EDN1",
  "gene": "UniProtKB:P05305",
  "gene_name": "Endothelin-1",
  "term_label": "extracellular space"
}